{
  "term_label": "Unknown biological process",
  "gene_symbol": "NAGK",
  "gene_name": "N-acetyl-D-glucosamine kinase",
  "gene": "UniProtKB:Q9UJ70",
  "term_id": "UNKNOWN:0002"
}